{
  "term_id": "GO:0008266",
  "term_label": "poly(U) RNA binding",
  "gene_symbol": "PABPC3",
  "gene_name": "Polyadenylate-binding protein 3",
  "gene": "UniProtKB:Q9H361"
}